{
  "gene": "UniProtKB:P13473",
  "term_label": "lysosomal membrane",
  "gene_name": "Lysosome-associated membrane glycoprotein 2",
  "term_id": "GO:0005765",
  "gene_symbol": "LAMP2"
}